{
  "term_id": "UNKNOWN:0003",
  "gene_symbol": "OR5AP2",
  "gene_name": "Olfactory receptor 5AP2",
  "gene": "UniProtKB:Q8NGF4",
  "term_label": "Unknown cellular component"
}